{
  "gene_name": "Ubiquitin carboxyl-terminal hydrolase 17-like protein 3",
  "term_label": "cytosol",
  "gene_symbol": "USP17L3",
  "term_id": "GO:0005829",
  "gene": "UniProtKB:A6NCW0"
}